{
  "gene_symbol": "SCO1",
  "term_id": "GO:0033617",
  "term_label": "mitochondrial respiratory chain complex IV assembly",
  "gene_name": "Protein SCO1 homolog, mitochondrial",
  "gene": "UniProtKB:O75880"
}